N-terminal protein amino acid deamination, from amino carbon [GO:0018058] (biological process) Sources: RESID:AA0127, RESID:AA0128, RESID:AA0129 Relationships: is a type of peptidyl-cysteine modification [GO:0018198]; is a type of protein deamination [GO:0018277]; is a type of N-terminal protein amino acid deamination [GO:0031363] Definition: The oxidative deamination of the alpha carbon of an encoded N-terminal amino acid, to form pyruvic acid retaining an amide bond between its 1-carboxyl group and the adjacent residue. The pyruvate 2-oxo group may become an enzyme active site, or it may be reduced to an alcohol.